potassium ion-transporting ATPase complex [GO:0031004] (cellular component) Relationships: is a type of cation-transporting ATPase complex [GO:0090533] References: PMID:10608856, PMID:9858692 Definition: Protein complex that carries out the reaction: ATP + H2O + K+(out) = ADP + phosphate + K+(in). It is a high affinity potassium uptake system. The E. coli complex consists of 4 proteins: KdpA is the potassium ion translocase, KdpB is the ATPase, and KdpC and KdpF seem to be involved in assembly and stabilization of the complex. Also known as: Kdp system complex